{
  "term_id": "GO:0006538",
  "gene": "UniProtKB:P49448",
  "gene_symbol": "GLUD2",
  "term_label": "L-glutamate catabolic process",
  "gene_name": "Glutamate dehydrogenase 2, mitochondrial"
}